{
  "gene": "UniProtKB:Q0D2K0",
  "gene_symbol": "NIPAL4",
  "term_label": "Unknown molecular function",
  "term_id": "UNKNOWN:0001",
  "gene_name": "Magnesium transporter NIPA4"
}